{
  "term_id": "GO:0007389",
  "gene_name": "T-box transcription factor TBX5",
  "gene_symbol": "TBX5",
  "term_label": "pattern specification process",
  "gene": "UniProtKB:Q99593"
}